serine-sulfate ammonia-lyase activity [GO:0050283] (molecular function) Definition: Catalysis of the reaction: L-serine O-sulfate + H2O = pyruvate + NH3 + sulfate. Sources: EC:4.3.1.10, MetaCyc:SERINE-SULFATE-AMMONIA-LYASE-RXN Relationships: is a type of ammonia-lyase activity [GO:0016841] Also known as: serine-sulphate ammonia-lyase activity, (L-SOS)lyase activity, L-serine-O-sulfate ammonia-lyase (pyruvate-forming)